{
  "gene": "UniProtKB:Q9HC57",
  "gene_symbol": "WFDC1",
  "term_id": "GO:0001558",
  "gene_name": "WAP four-disulfide core domain protein 1",
  "term_label": "regulation of cell growth"
}